{
  "gene_symbol": "DHRS1",
  "term_label": "Unknown molecular function",
  "gene_name": "Dehydrogenase_reductase SDR family member 1",
  "gene": "UniProtKB:Q96LJ7",
  "term_id": "UNKNOWN:0001"
}